{
  "term_id": "GO:0020037",
  "gene_name": "Sulfite oxidase, mitochondrial",
  "term_label": "heme binding",
  "gene": "UniProtKB:P51687",
  "gene_symbol": "SUOX"
}